{
  "gene_name": "Zinc finger protein 787",
  "gene": "UniProtKB:Q6DD87",
  "term_id": "GO:0005634",
  "term_label": "nucleus",
  "gene_symbol": "ZNF787"
}